{
  "term_id": "GO:0006954",
  "gene": "UniProtKB:Q9NZH6",
  "gene_symbol": "IL37",
  "gene_name": "Interleukin-37",
  "term_label": "inflammatory response"
}